{
  "gene_name": "Rho-associated protein kinase 2",
  "term_label": "Rho protein signal transduction",
  "gene_symbol": "ROCK2",
  "term_id": "GO:0007266",
  "gene": "UniProtKB:O75116"
}